{
  "gene_symbol": "LINC00308",
  "term_label": "Unknown biological process",
  "gene_name": "Putative uncharacterized protein encoded by LINC00308",
  "term_id": "UNKNOWN:0002",
  "gene": "UniProtKB:Q8TCZ7"
}